{
  "gene_symbol": "ZCCHC3",
  "gene_name": "Zinc finger CCHC domain-containing protein 3",
  "term_id": "GO:0051607",
  "gene": "UniProtKB:Q9NUD5",
  "term_label": "defense response to virus"
}